{
  "term_label": "Unknown biological process",
  "gene_symbol": "KRTAP5-2",
  "gene_name": "Keratin-associated protein 5-2",
  "term_id": "UNKNOWN:0002",
  "gene": "UniProtKB:Q701N4"
}